{
  "term_label": "endoplasmic reticulum exit site",
  "gene": "UniProtKB:A0A2R8YE69",
  "gene_name": "Uncharacterized protein",
  "gene_symbol": "A0A2R8YE69",
  "term_id": "GO:0070971"
}